{
  "term_id": "GO:0048259",
  "gene": "UniProtKB:Q6ZTN6",
  "gene_symbol": "ANKRD13D",
  "term_label": "regulation of receptor-mediated endocytosis",
  "gene_name": "Ankyrin repeat domain-containing protein 13D"
}